nuclear migration to embryo sac poles [GO:0023002] (biological process) Definition: Migration of the nuclei of the two-nucleate embryo sac to opposite poles of the cell. Sources: GOC:jid, GOC:mtg_plant, ISBN:047186840X Also known as: nuclear migration to female gametophyte poles, nuclear migration to megagametophyte poles, nucleus migration to embryo sac poles, nucleus migration to female gametophyte poles, nucleus migration to megagametophyte poles Relationships: is a type of GO:0009562